aspartyl-tRNA aminoacylation [GO:0006422] (biological process) Definition: The process of coupling aspartate to aspartyl-tRNA, catalyzed by aspartyl-tRNA synthetase. The aspartyl-tRNA synthetase is a class-II synthetase. The activated amino acid is transferred to the 3'-OH group of an aspartic acid accetping tRNA. Relationships: is a type of tRNA aminoacylation for protein translation [GO:0006418] Sources: GOC:mah, ISBN:0716730510 Subtypes: mitochondrial aspartyl-tRNA aminoacylation [GO:0070146]